{
  "term_label": "Unknown cellular component",
  "gene": "UniProtKB:Q8WXI3",
  "gene_symbol": "ASB10",
  "term_id": "UNKNOWN:0003",
  "gene_name": "Ankyrin repeat and SOCS box protein 10"
}